{
  "term_id": "GO:0005634",
  "term_label": "nucleus",
  "gene_name": "Zinc finger protein 254",
  "gene_symbol": "ZNF254",
  "gene": "UniProtKB:O75437"
}